{
  "term_label": "Unknown biological process",
  "gene": "UniProtKB:Q9BWS9",
  "gene_name": "Chitinase domain-containing protein 1",
  "gene_symbol": "CHID1",
  "term_id": "UNKNOWN:0002"
}